smoothened signaling pathway involved in ventral spinal cord interneuron specification [GO:0021775] (biological process) Also known as: hedgehog signaling pathway involved in ventral spinal cord interneuron specification, hh signaling pathway involved in ventral spinal cord interneuron specification, smoothened signalling pathway involved in ventral spinal cord interneuron specification Relationships: is a type of smoothened signaling pathway involved in ventral spinal cord patterning [GO:0021910]; is part of ventral spinal cord interneuron specification [GO:0021521] Definition: The series of molecular signals initiated by binding of a ligand to the transmembrane receptor smoothened in a precursor cell in the ventral spinal cord that contributes to the commitment of the precursor cell to an interneuron fate. References: PMID:11262869 Sources: GOC:cls, GOC:dgh, GOC:dph, GOC:jid, GO_REF:0000021